{
  "gene_name": "RuvB-like 2",
  "gene_symbol": "RUVBL2",
  "term_id": "GO:0006338",
  "term_label": "chromatin remodeling",
  "gene": "UniProtKB:Q9Y230"
}